{
  "term_label": "Unknown molecular function",
  "gene_symbol": "TG",
  "term_id": "UNKNOWN:0001",
  "gene_name": "Thyroglobulin",
  "gene": "UniProtKB:P01266"
}